{
  "gene_symbol": "KAT2B",
  "gene": "UniProtKB:Q92831",
  "term_id": "GO:0140672",
  "term_label": "ATAC complex",
  "gene_name": "Histone acetyltransferase KAT2B"
}